positive regulation of non-professional antigen presenting cell antigen processing and presentation [GO:0002621] (biological process) Also known as: up regulation of non-professional antigen presenting cell antigen processing and presentation, up-regulation of non-professional antigen presenting cell antigen processing and presentation, upregulation of non-professional antigen presenting cell antigen processing and presentation, activation of non-professional antigen presenting cell antigen processing and presentation, stimulation of non-professional antigen presenting cell antigen processing and presentation Sources: GOC:add Definition: Any process that activates or increases the frequency, rate, or extent of non-professional antigen presenting cell antigen processing and presentation. Relationships: is a type of positive regulation of antigen processing and presentation [GO:0002579]; is a type of GO:0002619; positively regulates non-professional antigen presenting cell antigen processing and presentation [GO:0002473]